{
  "gene_symbol": "NEDD4L",
  "term_label": "neuromuscular junction development",
  "gene": "UniProtKB:Q96PU5",
  "term_id": "GO:0007528",
  "gene_name": "E3 ubiquitin-protein ligase NEDD4-like"
}